{
  "gene_symbol": "RAB3B",
  "gene_name": "Ras-related protein Rab-3B",
  "gene": "UniProtKB:P20337",
  "term_label": "GTPase activity",
  "term_id": "GO:0003924"
}